{
  "term_id": "GO:0006357",
  "term_label": "regulation of transcription by RNA polymerase II",
  "gene_symbol": "ERF",
  "gene_name": "ETS domain-containing transcription factor ERF",
  "gene": "UniProtKB:P50548"
}